{
  "gene_name": "Killer cell immunoglobulin-like receptor 3DL3",
  "term_id": "GO:0002767",
  "gene": "UniProtKB:Q8N743",
  "term_label": "immune response-inhibiting cell surface receptor signaling pathway",
  "gene_symbol": "KIR3DL3"
}